{
  "gene_name": "Dipeptidyl peptidase 4",
  "gene": "UniProtKB:P27487",
  "gene_symbol": "DPP4",
  "term_id": "GO:0006508",
  "term_label": "proteolysis"
}